{
  "gene_name": "UPF0538 protein C2orf76",
  "term_id": "UNKNOWN:0002",
  "term_label": "Unknown biological process",
  "gene_symbol": "C2orf76",
  "gene": "UniProtKB:Q3KRA6"
}